ligase regulator activity [GO:0055103] (molecular function) Sources: GOC:BHF, GOC:rl Relationships: is a type of enzyme regulator activity [GO:0030234]; regulates ligase activity [GO:0016874] Subtypes: ligase inhibitor activity [GO:0055104], tRNA ligase activator activity [GO:0140733], SUMO ligase regulator activity [GO:0180016], glutamate-cysteine ligase regulator activity [GO:1990609] Definition: Binds to and modulates the activity of a ligase.